{
  "term_id": "GO:0004984",
  "gene": "UniProtKB:A0A3B3IT45",
  "gene_name": "Olfactory receptor",
  "term_label": "olfactory receptor activity",
  "gene_symbol": "OR51C1"
}